second mitotic wave involved in compound eye morphogenesis [GO:0016330] (BP) Relationships: is a type of GO:0000278; is part of compound eye morphogenesis [GO:0001745] Also known as: second mitotic wave during compound eye morphogenesis References: PMID:11257224 Definition: A discrete cell cycle in the third instar eye imaginal disc after progression of the morphogenetic furrow that contributes to compound eye morphogenesis. It is essential for generation of a sufficient pool of uncommitted cells to develop complete ommatidia.